{
  "gene_name": "Cytochrome c",
  "term_label": "mitochondrial intermembrane space",
  "gene": "UniProtKB:P99999",
  "term_id": "GO:0005758",
  "gene_symbol": "CYCS"
}